{
  "gene_name": "Adhesion G protein-coupled receptor F5",
  "gene": "UniProtKB:Q8IZF2",
  "term_label": "adenylate cyclase-activating G protein-coupled receptor signaling pathway",
  "gene_symbol": "ADGRF5",
  "term_id": "GO:0007189"
}